pyridine nucleotide salvage [GO:0019365] (biological process) Definition: Any process that generates a pyridine nucleotide, a nucleotide characterized by a pyridine derivative as a nitrogen base, from derivatives of them without de novo synthesis. Also known as: pyridine nucleotide cycling Subtypes: nicotinate nucleotide salvage [GO:0019358], NAD+ biosynthetic process via the salvage pathway [GO:0034355] Sources: GOC:jl Relationships: is_a GO:0019363; is a type of GO:0043173